{
  "gene_name": "Galactose mutarotase",
  "term_id": "GO:0006006",
  "gene": "UniProtKB:Q96C23",
  "gene_symbol": "GALM",
  "term_label": "glucose metabolic process"
}